heat shock protein binding [GO:0031072] (molecular function) Relationships: is a type of GO:0005515 Definition: Binding to a heat shock protein, a protein synthesized or activated in response to heat shock. Subtypes: Hsp70 protein binding [GO:0030544], Hsp27 protein binding [GO:0051008], Hsp90 protein binding [GO:0051879] Sources: GOC:mah, GOC:vw